cone photoreceptor disc membrane [GO:0120201] (cellular component) Relationships: is a type of ciliary membrane [GO:0060170]; is a type of photoreceptor disc membrane [GO:0097381] References: PMID:19501669, PMID:26574505, PMID:6771304 Sources: GOC:krc, GOC:pde Definition: Stack of disc membranes located inside a cone photoreceptor outer segment, and containing densely packed molecules of opsin photoreceptor proteins that traverse the lipid bilayer. Cone disc membranes arise as evaginations of the ciliary membrane during the development of the cone outer segment and remain contiguous with the ciliary membrane.